{
  "term_label": "alpha-ketoglutarate transmembrane transporter activity",
  "gene": "UniProtKB:Q13183",
  "term_id": "GO:0015139",
  "gene_name": "Solute carrier family 13 member 2",
  "gene_symbol": "SLC13A2"
}